response to very low fluence red light stimulus [GO:0010203] (biological process) Definition: Any process that results in a change in state or activity of a cell or an organism (in terms of movement, secretion, enzyme production, gene expression, etc.) as a result of a very low fluence red light stimulus. Red light is electromagnetic radiation of wavelength of 580-700nm. Very low fluence red light is defined in this case as short pulses of red light followed by darkness, providing light levels of less than 0.001 mmol/m2/sec. Sources: GOC:mtg_far_red, GOC:sm Relationships: is a type of response to red light [GO:0010114]; is a type of GO:0055122